{
  "gene_symbol": "MPG",
  "gene_name": "DNA-3-methyladenine glycosylase",
  "term_label": "Unknown cellular component",
  "gene": "UniProtKB:P29372",
  "term_id": "UNKNOWN:0003"
}